{
  "term_id": "UNKNOWN:0002",
  "gene_name": "Nuclear factor NF-kappa-B p105 subunit",
  "gene_symbol": "NFKB1",
  "gene": "UniProtKB:P19838",
  "term_label": "Unknown biological process"
}